{
  "gene_symbol": "CALR",
  "gene": "UniProtKB:P27797",
  "term_id": "GO:0036503",
  "term_label": "ERAD pathway",
  "gene_name": "Calreticulin"
}